{
  "gene_symbol": "CD200R1",
  "term_label": "external side of plasma membrane",
  "term_id": "GO:0009897",
  "gene": "UniProtKB:Q8TD46",
  "gene_name": "Cell surface glycoprotein CD200 receptor 1"
}